{
  "gene_name": "MORC family CW-type zinc finger protein 3",
  "gene": "UniProtKB:Q14149",
  "term_id": "GO:0016605",
  "gene_symbol": "MORC3",
  "term_label": "PML body"
}